aminocarboxymuconate-semialdehyde decarboxylase activity [GO:0001760] (molecular function) Definition: Catalysis of the reaction: 2-amino-3-carboxymuconate 6-semialdehyde + H+ = 2-aminomuconate 6-semialdehyde + CO2. Also known as: ACMSD activity, 2-amino-3-(3-oxoprop-1-en-1-yl)but-2-enedioate carboxy-lyase (2-aminomuconate-semialdehyde-forming), 2-amino-3-(3-oxoprop-1-en-1-yl)but-2-enedioate carboxy-lyase activity, 2-amino-3-(3-oxoprop-2-enyl)but-2-enedioate carboxy-lyase activity, alpha-amino-beta-carboxymuconate-epsilon-semialdehade decarboxylase activity, alpha-amino-beta-carboxymuconate-epsilon-semialdehyde beta-decarboxylase activity, picolinic acid carboxylase activity, picolinic acid decarboxylase activity Relationships: is a type of GO:0016831 Sources: EC:4.1.1.45, RHEA:16557